{
  "term_label": "Unknown cellular component",
  "gene": "UniProtKB:Q92785",
  "term_id": "UNKNOWN:0003",
  "gene_symbol": "DPF2",
  "gene_name": "Zinc finger protein ubi-d4"
}